negative regulation of purine nucleoside transport [GO:0032247] (biological process) Relationships: is a type of negative regulation of nucleoside transport [GO:0032243]; is a type of regulation of purine nucleoside transport [GO:0032245] Subtypes: negative regulation of adenosine transport [GO:0032250], negative regulation of inosine transport [GO:0035343] Also known as: down regulation of purine nucleoside transport, down-regulation of purine nucleoside transport, downregulation of purine nucleoside transport, inhibition of purine nucleoside transport Definition: Any process that stops, prevents, or reduces the frequency, rate or extent of the directed movement of a purine nucleoside into, out of or within a cell, or between cells, by means of some agent such as a transporter or pore. Sources: GOC:mah